{
  "term_label": "regulation of transcription by RNA polymerase II",
  "gene": "UniProtKB:Q86Y25",
  "term_id": "GO:0006357",
  "gene_symbol": "ZNF354C",
  "gene_name": "Zinc finger protein 354C"
}